{
  "gene_symbol": "SLFN11",
  "term_id": "UNKNOWN:0003",
  "term_label": "Unknown cellular component",
  "gene_name": "Schlafen family member 11",
  "gene": "UniProtKB:Q7Z7L1"
}